{
  "term_label": "Unknown molecular function",
  "gene_symbol": "TMEM176A",
  "gene_name": "Transmembrane protein 176A",
  "term_id": "UNKNOWN:0001",
  "gene": "UniProtKB:Q96HP8"
}